{
  "gene": "UniProtKB:Q5T1V6",
  "gene_name": "Probable ATP-dependent RNA helicase DDX59",
  "gene_symbol": "DDX59",
  "term_label": "Unknown biological process",
  "term_id": "UNKNOWN:0002"
}